{
  "gene_name": "Alpha-actinin-1",
  "term_label": "actin cytoskeleton organization",
  "gene_symbol": "ACTN1",
  "gene": "UniProtKB:P12814",
  "term_id": "GO:0030036"
}